outer dynein arm assembly [GO:0036158] (biological process) References: PMID:19944400 Sources: GOC:BHF, GOC:vk Definition: The aggregation, arrangement and bonding together of a set of components to form an axonemal dynein outer arm, an outer arm structure present on the outer doublet microtubules of ciliary and flagellar axonemes. Also known as: ODA assembly Relationships: is a type of GO:0070286